{
  "gene_name": "Terminal nucleotidyltransferase 5A",
  "term_id": "UNKNOWN:0003",
  "gene_symbol": "TENT5A",
  "term_label": "Unknown cellular component",
  "gene": "UniProtKB:Q96IP4"
}